{
  "term_label": "Unknown biological process",
  "gene_symbol": "GASK1A",
  "gene_name": "Golgi-associated kinase 1A",
  "gene": "UniProtKB:Q9UFP1",
  "term_id": "UNKNOWN:0002"
}